{
  "gene_symbol": "PTPRN",
  "gene_name": "Receptor-type tyrosine-protein phosphatase-like N",
  "term_id": "GO:0051046",
  "term_label": "regulation of secretion",
  "gene": "UniProtKB:Q16849"
}